{
  "gene": "UniProtKB:P10809",
  "term_label": "apoptotic mitochondrial changes",
  "term_id": "GO:0008637",
  "gene_name": "60 kDa heat shock protein, mitochondrial",
  "gene_symbol": "HSPD1"
}